tRNA (guanine(6)-N2)-methyltransferase activity [GO:0160117] (molecular function) Relationships: is a type of N-methyltransferase activity [GO:0008170]; is a type of tRNA (guanine) methyltransferase activity [GO:0016423] Definition: Catalysis of the reaction: guanosine(6) in tRNA + S-adenosyl-L-methionine = H+ + N(2)-methylguanosine(6) in tRNA + S-adenosyl-L-homocysteine. References: PMID:34669960 Sources: EC:2.1.1.256 Also known as: m(2)G6 methyltransferase, methyltransferase Trm14